shoot organ boundary specification [GO:0090470] (biological process) References: PMID:18757555 Definition: The process in which the basal boundary between the stem and both vegetative and reproductive organs are established and maintained. Relationships: is a type of GO:0090691